{
  "term_label": "3'-UTR-mediated mRNA destabilization",
  "term_id": "GO:0061158",
  "gene_name": "Protein NYNRIN",
  "gene": "UniProtKB:Q9P2P1",
  "gene_symbol": "NYNRIN"
}